{
  "gene": "UniProtKB:Q9H5Z6",
  "gene_symbol": "FAM124B",
  "term_label": "Unknown molecular function",
  "gene_name": "Protein FAM124B",
  "term_id": "UNKNOWN:0001"
}